{
  "term_id": "GO:0003724",
  "gene_name": "ATP-dependent RNA helicase DDX3X",
  "gene_symbol": "DDX3X",
  "term_label": "RNA helicase activity",
  "gene": "UniProtKB:O00571"
}